{
  "gene_symbol": "OPRK1",
  "gene_name": "Kappa-type opioid receptor",
  "gene": "UniProtKB:P41145",
  "term_label": "neuropeptide signaling pathway",
  "term_id": "GO:0007218"
}